{
  "term_label": "plasma membrane",
  "gene": "UniProtKB:Q8NGE8",
  "term_id": "GO:0005886",
  "gene_name": "Olfactory receptor 4D9",
  "gene_symbol": "OR4D9"
}